enucleate erythrocyte maturation [GO:0043354] (biological process) Relationships: is a type of erythrocyte maturation [GO:0043249]; BFO_0000050 enucleate erythrocyte development [GO:0048822] Sources: GOC:go_curators Also known as: enucleate RBC maturation, enucleate red blood cell maturation Definition: A developmental process, independent of morphogenetic (shape) change, that is required for an enucleate erythrocyte to attain its fully functional state. An enucleate erythrocyte is an erythrocyte without a nucleus.